{
  "term_id": "GO:0004117",
  "gene_symbol": "PDE1A",
  "term_label": "calmodulin-activated dual specificity 3',5'-cyclic-GMP, 3',5'-cyclic-AMP phosphodiesterase activity",
  "gene_name": "Dual specificity calcium_calmodulin-dependent 3',5'-cyclic nucleotide phosphodiesterase 1A",
  "gene": "UniProtKB:P54750"
}